{
  "gene_symbol": "SERPINA7",
  "term_label": "extracellular space",
  "term_id": "GO:0005615",
  "gene_name": "Thyroxine-binding globulin",
  "gene": "UniProtKB:P05543"
}